{
  "term_id": "GO:0050803",
  "gene_symbol": "SLC17A6",
  "gene": "UniProtKB:Q9P2U8",
  "gene_name": "Vesicular glutamate transporter 2",
  "term_label": "regulation of synapse structure or activity"
}